{
  "gene": "UniProtKB:Q9UKG4",
  "term_id": "GO:0005886",
  "term_label": "plasma membrane",
  "gene_symbol": "SLC13A4",
  "gene_name": "Solute carrier family 13 member 4"
}